acyl-CoA ceramide synthase complex [GO:0061576] (cellular component) References: PMID:15692566 Sources: GOC:dph Definition: A protein complex that catalyzes the reaction acyl-CoA + sphingosine = CoA + N-acylsphingosine. In S. cerevisiae it contains three subunits: lag1, lac1 and lip1. Relationships: is_a catalytic complex [GO:1902494]